{
  "term_label": "microtubule cytoskeleton",
  "gene": "UniProtKB:Q9UHD8",
  "gene_symbol": "SEPTIN9",
  "gene_name": "Septin-9",
  "term_id": "GO:0015630"
}